peptidyl-lysine methylation [GO:0018022] (biological process) Sources: GOC:ai Subtypes: peptidyl-lysine trimethylation [GO:0018023], peptidyl-lysine monomethylation [GO:0018026], peptidyl-lysine dimethylation [GO:0018027] Definition: The methylation of peptidyl-lysine to form either the mono-, di- or trimethylated derivative. Relationships: is a type of GO:0006479; is a type of GO:0018205